{
  "term_label": "histone binding",
  "gene_symbol": "YEATS2",
  "gene_name": "YEATS domain-containing protein 2",
  "term_id": "GO:0042393",
  "gene": "UniProtKB:Q9ULM3"
}